{
  "gene_symbol": "COG2",
  "gene_name": "Conserved oligomeric Golgi complex subunit 2",
  "term_id": "UNKNOWN:0001",
  "gene": "UniProtKB:Q14746",
  "term_label": "Unknown molecular function"
}